positive regulation of bone remodeling [GO:0046852] (biological process) Definition: Any process that activates or increases the frequency, rate or extent of bone remodeling. Sources: GOC:ai Also known as: positive regulation of bone remodelling, up regulation of bone remodeling, up-regulation of bone remodeling, upregulation of bone remodeling, activation of bone remodeling, stimulation of bone remodeling Relationships: is a type of GO:0034105; is a type of GO:0046850; positively regulates bone remodeling [GO:0046849]